{
  "term_label": "plasma membrane",
  "gene_name": "Protein crumbs homolog 1",
  "gene_symbol": "CRB1",
  "term_id": "GO:0005886",
  "gene": "UniProtKB:P82279"
}